negative regulation of heart rate [GO:0010459] (biological process) Definition: Any process that stops, prevents or reduces the frequency or rate of heart contraction. Sources: GOC:dph, GOC:tb Relationships: is a type of regulation of heart rate [GO:0002027]; is a type of negative regulation of heart contraction [GO:0045822] Subtypes: negative regulation of heart rate involved in baroreceptor response to increased systemic arterial blood pressure [GO:0001985], GO:0003063